{
  "gene_name": "Glycine N-acyltransferase",
  "term_id": "GO:0006544",
  "gene_symbol": "GLYAT",
  "term_label": "glycine metabolic process",
  "gene": "UniProtKB:Q6IB77"
}